{
  "gene_symbol": "POLR2D",
  "term_id": "GO:0005665",
  "term_label": "RNA polymerase II, core complex",
  "gene_name": "DNA-directed RNA polymerase II subunit RPB4",
  "gene": "UniProtKB:O15514"
}